positive regulation of synaptic vesicle membrane organization [GO:1901634] (biological process) Subtypes: positive regulation of synaptic vesicle fusion to presynaptic active zone membrane [GO:0031632] Relationships: is a type of GO:0051130; is a type of GO:1901632; positively regulates synaptic vesicle membrane organization [GO:0048499] References: PMID:22426000 Sources: GOC:TermGenie Also known as: positive regulation of synaptic vesicle membrane organisation, up regulation of synaptic vesicle membrane organisation, up regulation of synaptic vesicle membrane organization, up-regulation of synaptic vesicle membrane organisation, up-regulation of synaptic vesicle membrane organization, upregulation of synaptic vesicle membrane organisation, upregulation of synaptic vesicle membrane organization, activation of SLMV biogenesis, activation of synaptic vesicle membrane organisation, activation of synaptic vesicle membrane organization, positive regulation of SLMV biogenesis, up regulation of SLMV biogenesis, up-regulation of SLMV biogenesis, upregulation of SLMV biogenesis, activation of synaptic vesicle membrane organization and biogenesis, positive regulation of synaptic vesicle membrane organization and biogenesis, up regulation of synaptic vesicle membrane organization and biogenesis, up-regulation of synaptic vesicle membrane organization and biogenesis, upregulation of synaptic vesicle membrane organization and biogenesis Definition: Any process that activates or increases the frequency, rate or extent of synaptic vesicle membrane organization.